23S rRNA pseudouridine(2605) synthase activity [GO:0160139] (molecular function) Relationships: is a type of rRNA pseudouridine synthase activity [GO:0120159] Sources: EC:5.4.99.22, RHEA:42520 Definition: Catalysis of the reaction: uridine(2605) in 23S rRNA = pseudouridine(2605) in 23S rRNA.